regulation of deacetylase activity [GO:0150065] (BP) References: PMID:19457097 Sources: GOC:aruk, GOC:bc Relationships: is a type of regulation of catalytic activity [GO:0050790]; regulates deacetylase activity [GO:0019213] Definition: Any process that modulates the frequency, rate or extent of deacetylase activity. Subtypes: positive regulation of deacetylase activity [GO:0090045]